NAD-dependent protein biotinidase activity [GO:0106420] (molecular function) Definition: Catalysis of the reaction: H2O + N6-biotinyl-L-lysyl-[protein] + NAD+ = 2''-O-biotinyl-ADP-D-ribose + L-lysyl-[protein] + nicotinamide. Relationships: is a type of acyltransferase activity, transferring groups other than amino-acyl groups [GO:0016747] References: PMID:25525879 Sources: RHEA:70479